equatorial microtubule organizing center [GO:0000923] (cellular component) Definition: A microtubule organizing center formed by a band of gamma-tubulin that is recruited to a circumferential band of F-actin at the midpoint of a cell and which nucleates microtubules from the cell division site at the end of mitosis. References: PMID:11792817 Also known as: EMTOC, equatorial microtubule organising centre Relationships: is a type of microtubule organizing center [GO:0005815]; is part of cell division site [GO:0032153]